regulation of viral DNA genome packaging via site-specific sequence recognition [GO:1905137] (biological process) Subtypes: positive regulation of viral DNA genome packaging via site-specific sequence recognition [GO:1905138] Definition: Any process that modulates the frequency, rate or extent of viral DNA genome packaging via site-specific sequence recognition. References: PMID:24711378 Sources: GOC:TermGenie, GO_REF:0000058 Relationships: is a type of GO:1903900; regulates viral DNA genome packaging via site-specific sequence recognition [GO:0098035]